{
  "gene_name": "Lysine--tRNA ligase",
  "term_id": "GO:0005739",
  "gene_symbol": "KARS1",
  "gene": "UniProtKB:Q15046",
  "term_label": "mitochondrion"
}